B800-850 antenna complex [GO:0030082] (cellular component) Relationships: is a type of protein-containing complex [GO:0032991]; is part of light-harvesting complex, peripheral complex [GO:0030079] Definition: Protein-pigment complex that absorbs light at 800 and 850 nm; is peripherally associated to the bacterial reaction center; transfers excitation energy to the B875 antenna complex. Sources: GOC:kd, GOC:lr Also known as: LH2 complex, light harvesting complex II